{
  "gene": "UniProtKB:Q14202",
  "gene_symbol": "ZMYM3",
  "gene_name": "Zinc finger MYM-type protein 3",
  "term_label": "Unknown biological process",
  "term_id": "UNKNOWN:0002"
}